{
  "gene_symbol": "ZBTB6",
  "gene": "UniProtKB:Q15916",
  "gene_name": "Zinc finger and BTB domain-containing protein 6",
  "term_id": "GO:0000978",
  "term_label": "RNA polymerase II cis-regulatory region sequence-specific DNA binding"
}